{
  "gene": "UniProtKB:Q13103",
  "gene_name": "Secreted phosphoprotein 24",
  "term_id": "UNKNOWN:0003",
  "gene_symbol": "SPP2",
  "term_label": "Unknown cellular component"
}